{
  "term_label": "lipopolysaccharide catabolic process",
  "gene": "UniProtKB:P28039",
  "gene_name": "Acyloxyacyl hydrolase",
  "gene_symbol": "AOAH",
  "term_id": "GO:0009104"
}